{
  "term_label": "serine-type endopeptidase activity",
  "gene": "UniProtKB:P10323",
  "term_id": "GO:0004252",
  "gene_symbol": "ACR",
  "gene_name": "Acrosin"
}